{
  "gene_symbol": "KLHDC8A",
  "term_label": "Unknown biological process",
  "term_id": "UNKNOWN:0002",
  "gene_name": "Kelch domain-containing protein 8A",
  "gene": "UniProtKB:Q8IYD2"
}